attachment of telomeric heterochromatin to nuclear envelope [GO:0140698] (biological process) References: PMID:31635174 Relationships: is a type of chromosome attachment to the nuclear envelope [GO:0097240] Definition: The process in which physical connections are formed between sub-telomeric heterochromatin and the nuclear envelope facilitating bouquet formation. Also known as: attachment of telomeres to nuclear envelope, attachment of telomeric chromatin to nuclear envelope, heterochromatin organization